regulation of chromosome organization [GO:0033044] (BP) Also known as: regulation of chromosome organisation, regulation of chromosome organization and biogenesis Subtypes: regulation of sister chromatid cohesion [GO:0007063], regulation of telomere maintenance [GO:0032204], regulation of sister chromatid segregation [GO:0033045], GO:0060623, GO:0062123, regulation of synaptonemal complex assembly [GO:0090173], GO:0090234, regulation of oocyte karyosome formation [GO:0120313], regulation of replication fork arrest at rDNA repeats [GO:1902681], GO:2001251, positive regulation of chromosome organization [GO:2001252] Definition: Any process that modulates the frequency, rate or extent of a process involved in the formation, arrangement of constituent parts, or disassembly of a chromosome. Relationships: is_a GO:0033043; regulates chromosome organization [GO:0051276] Sources: GOC:mah